{
  "term_id": "GO:0001881",
  "gene_name": "Rab15 effector protein",
  "term_label": "receptor recycling",
  "gene": "UniProtKB:Q6BDI9",
  "gene_symbol": "REP15"
}